{
  "gene_symbol": "SLC26A2",
  "gene": "UniProtKB:P50443",
  "term_id": "GO:0015116",
  "term_label": "sulfate transmembrane transporter activity",
  "gene_name": "Sulfate transporter"
}